regulation of tumor necrosis factor (ligand) superfamily member 11 production [GO:2000307] (BP) Definition: Any process that modulates the frequency, rate or extent of tumor necrosis factor (ligand) superfamily member 11 production. Relationships: is a type of regulation of tumor necrosis factor superfamily cytokine production [GO:1903555]; regulates tumor necrosis factor (ligand) superfamily member 11 production [GO:0072535] Subtypes: negative regulation of tumor necrosis factor (ligand) superfamily member 11 production [GO:2000308], positive regulation of tumor necrosis factor (ligand) superfamily member 11 production [GO:2000309] Sources: GOC:BHF, GOC:mah Also known as: regulation of RANKL production, regulation of TNFSF11 production